{
  "gene": "UniProtKB:Q9ULE6",
  "term_label": "protein tyrosine phosphatase activity",
  "gene_symbol": "PALD1",
  "term_id": "GO:0004725",
  "gene_name": "Paladin"
}